{
  "term_label": "lysosomal HOPS complex",
  "gene_symbol": "VPS39",
  "term_id": "GO:1902501",
  "gene": "UniProtKB:Q96JC1",
  "gene_name": "Vam6_Vps39-like protein"
}